{
  "gene_name": "Tyrosine-protein kinase JAK2",
  "term_label": "growth hormone receptor binding",
  "gene": "UniProtKB:O60674",
  "gene_symbol": "JAK2",
  "term_id": "GO:0005131"
}